{
  "gene": "UniProtKB:Q01432",
  "gene_name": "AMP deaminase 3",
  "term_id": "GO:0003876",
  "term_label": "AMP deaminase activity",
  "gene_symbol": "AMPD3"
}